{
  "gene": "UniProtKB:O95397",
  "gene_name": "Putative protein PLEKHA9",
  "gene_symbol": "PLEKHA8P1",
  "term_label": "intermembrane lipid transfer",
  "term_id": "GO:0120009"
}